{
  "gene_name": "Lactosylceramide alpha-2,3-sialyltransferase",
  "gene": "UniProtKB:Q9UNP4",
  "gene_symbol": "ST3GAL5",
  "term_id": "UNKNOWN:0003",
  "term_label": "Unknown cellular component"
}